immune system process [GO:0002376] (biological process) Relationships: is a type of biological_process [GO:0008150] Note: Note that this term is a direct child of 'biological_process ; GO:0008150' because some immune system processes are types of cellular process (GO:0009987), whereas others are types of multicellular organism process (GO:0032501). Sources: GOC:add, GO_REF:0000022 Subtypes: leukocyte homeostasis [GO:0001776], GO:0002200, immune effector process [GO:0002252], activation of immune response [GO:0002253], myeloid cell homeostasis [GO:0002262], B cell selection [GO:0002339], antigen sampling in mucosal-associated lymphoid tissue [GO:0002404], production of molecular mediator of immune response [GO:0002440], tolerance induction [GO:0002507], GO:0002520, GO:0006955, antigen processing and presentation [GO:0019882], GO:0031294, hemocyte proliferation [GO:0035172], GO:0042386, T cell selection [GO:0045058], leukocyte activation [GO:0045321], leukocyte migration [GO:0050900], immunological memory process [GO:0090713] Definition: Any process involved in the development or functioning of the immune system, an organismal system for calibrated responses to potential internal or invasive threats. Regulation: regulated by regulation of immune system process [GO:0002682]; negatively regulated by GO:0002683; positively regulated by positive regulation of immune system process [GO:0002684]